{
  "term_label": "nuclear envelope",
  "gene_symbol": "SUN1",
  "gene": "UniProtKB:O94901",
  "gene_name": "SUN domain-containing protein 1",
  "term_id": "GO:0005635"
}